maternal specification of dorsal/ventral axis, oocyte, germ-line encoded [GO:0007311] (biological process) Sources: GOC:dph, GOC:mtg_sensu, GOC:tb, ISBN:0879694238 Also known as: maternal determination of dorsal/ventral axis, oocyte, germ-line encoded, maternal specification of dorsal-ventral axis, oocyte, germ-line encoded, maternal specification of dorsoventral axis, oocyte, germ-line encoded Relationships: is a type of oocyte dorsal/ventral axis specification [GO:0007310] Definition: Polarization of the oocyte along the dorsal-ventral axis, by a gene product encoded by cells of the germ line. An example of this is found in Drosophila melanogaster.